{
  "term_id": "UNKNOWN:0001",
  "gene_symbol": "TATDN3",
  "gene_name": "Putative deoxyribonuclease TATDN3",
  "gene": "UniProtKB:Q17R31",
  "term_label": "Unknown molecular function"
}